{
  "term_id": "UNKNOWN:0002",
  "gene_symbol": "MRPS26",
  "gene_name": "Small ribosomal subunit protein mS26",
  "term_label": "Unknown biological process",
  "gene": "UniProtKB:Q9BYN8"
}